{
  "term_id": "GO:0007420",
  "gene": "UniProtKB:O95197",
  "term_label": "brain development",
  "gene_symbol": "RTN3",
  "gene_name": "Reticulon-3"
}